{
  "gene": "UniProtKB:P09565",
  "term_label": "Unknown cellular component",
  "gene_symbol": "GIG44",
  "term_id": "UNKNOWN:0003",
  "gene_name": "Putative insulin-like growth factor 2-associated protein"
}